{
  "term_label": "regulation of transcription by RNA polymerase II",
  "gene_symbol": "ZNF575",
  "term_id": "GO:0006357",
  "gene_name": "Zinc finger protein 575",
  "gene": "UniProtKB:Q86XF7"
}